insulin-like growth factor receptor activity [GO:0005010] (molecular function) Note: Note that this term represents an activity and not a gene product, and should only be used when the receptor binds the ligand IGF. For receptors that bind other growth factors, consider annotating to other terms under 'transmembrane signaling receptor activity ; GO:0004888. Definition: Combining with insulin-like growth factor receptor ligand and transmitting the signal across the plasma membrane to initiate a change in cell activity. Also known as: IGF receptor activity, IGF-activated receptor activity, insulin-like growth factor-activated receptor activity Relationships: is a type of GO:0004714; is part of GO:0048009; has part GO:0005520 Sources: GOC:mah